interleukin-1-mediated signaling pathway [GO:0070498] (biological process) Also known as: IL-1-mediated signaling pathway, interleukin-1-mediated signalling pathway, IL-1 alpha-mediated signaling pathway, IL-1 beta-mediated signaling pathway, interleukin-1 alpha-mediated signaling pathway, interleukin-1 beta-mediated signaling pathway Regulation: regulated by regulation of interleukin-1-mediated signaling pathway [GO:2000659]; RO_0002212 by negative regulation of interleukin-1-mediated signaling pathway [GO:2000660]; positively regulated by positive regulation of interleukin-1-mediated signaling pathway [GO:2000661] Sources: GOC:BHF, GOC:mah, GOC:signaling Definition: The series of molecular signals initiated by interleukin-1 binding to its receptor on the surface of a target cell, and ending with the regulation of a downstream cellular process, e.g. transcription. Relationships: is a type of GO:0019221; is part of cellular response to interleukin-1 [GO:0071347]